{
  "gene": "UniProtKB:P41226",
  "term_label": "ISG15-protein conjugation",
  "term_id": "GO:0032020",
  "gene_name": "Ubiquitin-like modifier-activating enzyme 7",
  "gene_symbol": "UBA7"
}